negative regulation of endosome to plasma membrane protein transport [GO:1905750] (biological process) Definition: Any process that stops, prevents or reduces the frequency, rate or extent of endosome to plasma membrane protein transport. Also known as: down regulation of endosome to plasma membrane protein transport, down-regulation of endosome to plasma membrane protein transport, downregulation of endosome to plasma membrane protein transport, inhibition of endosome to plasma membrane protein transport References: PMID:22869721 Sources: GOC:TermGenie, GO_REF:0000058 Relationships: is a type of GO:0090317; is_a negative regulation of protein localization to plasma membrane [GO:1903077]; is a type of regulation of endosome to plasma membrane protein transport [GO:1905749]; is a type of negative regulation of endocytic recycling [GO:2001136]; negatively regulates endosome to plasma membrane protein transport [GO:0099638]